{
  "term_id": "UNKNOWN:0002",
  "term_label": "Unknown biological process",
  "gene_name": "Zinc finger Ran-binding domain-containing protein 2",
  "gene": "UniProtKB:O95218",
  "gene_symbol": "ZRANB2"
}